octopamine signaling pathway [GO:0071927] (biological process) References: PMID:15355245 Sources: GOC:mah Regulation: regulated by GO:2000128; negatively regulated by negative regulation of octopamine signaling pathway [GO:2000129]; positively regulated by positive regulation of octopamine signaling pathway [GO:2000130] Also known as: octopamine signalling pathway Definition: The series of molecular signals generated as a consequence of octopamine binding to a cell surface receptor. Subtypes: octopamine signaling pathway involved in response to food [GO:0071935], positive regulation of fatty acid beta-oxidation by octopamine signaling pathway [GO:1904122] Relationships: is a type of GO:0007211